{
  "gene_symbol": "DNAAF10",
  "gene_name": "Dynein axonemal assembly factor 10",
  "gene": "UniProtKB:Q96MX6",
  "term_id": "UNKNOWN:0003",
  "term_label": "Unknown cellular component"
}